negative regulation of excitatory synapse assembly [GO:1904890] (biological process) Sources: GOC:PARL, GOC:TermGenie, GOC:bf, GO_REF:0000058 Relationships: is a type of GO:0051964; is_a regulation of excitatory synapse assembly [GO:1904889]; negatively regulates excitatory synapse assembly [GO:1904861] Definition: Any process that stops, prevents or reduces the frequency, rate or extent of excitatory synapse assembly. Also known as: down regulation of excitatory synapse assembly, down regulation of excitatory synapse formation, down-regulation of excitatory synapse assembly, down-regulation of excitatory synapse formation, downregulation of excitatory synapse assembly, downregulation of excitatory synapse formation, negative regulation of excitatory synapse formation, inhibition of excitatory synapse assembly, inhibition of excitatory synapse formation